{
  "term_id": "GO:0061630",
  "gene_name": "Tripartite motif-containing protein 5",
  "term_label": "ubiquitin protein ligase activity",
  "gene": "UniProtKB:Q9C035",
  "gene_symbol": "TRIM5"
}